{
  "gene": "UniProtKB:Q8NDT2",
  "term_id": "GO:0005634",
  "gene_symbol": "RBM15B",
  "gene_name": "Putative RNA-binding protein 15B",
  "term_label": "nucleus"
}